meiotic spindle midzone assembly [GO:0051257] (biological process) Definition: The formation of the spindle midzone, the area in the center of the spindle where the spindle microtubules from opposite poles overlap, as a part of the process of meiosis. Sources: GOC:ai, GOC:expert_rg, GOC:tb Also known as: meiotic spindle midzone biogenesis, meiotic spindle midzone biosynthesis, meiotic spindle midzone formation, spindle midzone assembly involved in meiosis, spindle midzone biogenesis involved in meiosis, spindle midzone biosynthesis involved in meiosis, spindle midzone formation involved in meiosis Relationships: is a type of spindle midzone assembly [GO:0051255]; is a type of meiotic cell cycle process [GO:1903046]; is part of meiotic nuclear division [GO:0140013]